aminoglycoside antibiotic biosynthetic process [GO:0030648] (biological process) Also known as: aminoglycoside antibiotic anabolism, aminoglycoside antibiotic biosynthesis, aminoglycoside antibiotic formation, aminoglycoside antibiotic synthesis Relationships: is a type of glycoside biosynthetic process [GO:0016138]; is a type of antibiotic biosynthetic process [GO:0017000] Definition: The chemical reactions and pathways resulting in the formation of an aminoglycoside antibiotic, any member of a group of broad spectrum antibiotics, of similar toxicity and pharmacology, that contain an aminodeoxysugar, an amino- or guanidino-substituted inositol ring, and one or more residues of other sugars. The group includes streptomycin, neomycin, framycetin, kanamycin, paromomycin, and gentamicin. Subtypes: streptomycin biosynthetic process [GO:0019872], gentamycin biosynthetic process [GO:1901130], kanamycin biosynthetic process [GO:1901133], vistamycin biosynthetic process [GO:1901152], GO:1901155, neomycin biosynthetic process [GO:1901158], daunorubicin biosynthetic process [GO:1901771] Sources: GOC:mah, ISBN:0198506732